viral translational frameshifting [GO:0075523] (biological process) Also known as: ribosomal frameshifting involved in viral translation Definition: A process which occurs during viral translation, which involves a translational recoding mechanism called programmed ribosomal frameshifting. This causes the ribosome to alter its reading of the mRNA to an a different open reading frame to produce alternate viral proteins. Note: This term is intended to annotate gene products involved in the process of viral translational frameshifting, not viral proteins produced by this translation process. Relationships: is a type of viral process [GO:0016032]; is part of viral translation [GO:0019081] References: PMID:24825891, PMID:8852897 Sources: GOC:bf, GOC:ch, GOC:jl, VZ:860